response to other organism [GO:0051707] (biological process) Sources: GOC:ai Subtypes: response to protozoan [GO:0001562], GO:0002213, defense response to nematode [GO:0002215], response to oomycetes [GO:0002239], response to symbiont [GO:0009608], GO:0009615, response to bacterium [GO:0009617], response to fungus [GO:0009620], GO:0009624, response to insect [GO:0009625], response to host [GO:0075136], response to herbivore [GO:0080027], GO:0098542, detection of other organism [GO:0098543] Relationships: is_a GO:0043207; is a type of biological process involved in interspecies interaction between organisms [GO:0044419] Definition: Any process that results in a change in state or activity of a cell or an organism (in terms of movement, secretion, enzyme production, gene expression, etc.) as a result of a stimulus from another living organism.